pancreatic D cell differentiation [GO:0003311] (biological process) Definition: The process in which relatively unspecialized cells acquire specialized structural and functional features that characterize a pancreatic delta cell. A delta cell is a cell of the pancreas that produces somatostatin. References: PMID:11076772 Sources: GOC:dph Relationships: is a type of enteroendocrine cell differentiation [GO:0035883]; is a type of neuroendocrine cell differentiation [GO:0061101]; is part of endocrine pancreas development [GO:0031018] Also known as: pancreatic delta cell differentiation